{
  "gene": "UniProtKB:Q8NE09",
  "term_label": "G-protein alpha-subunit binding",
  "term_id": "GO:0001965",
  "gene_symbol": "RGS22",
  "gene_name": "Regulator of G-protein signaling 22"
}